trans-Golgi network transport vesicle membrane [GO:0012510] (cellular component) Definition: The lipid bilayer surrounding a vesicle transporting substances between the trans-Golgi network and other parts of the cell. Sources: GOC:ai Relationships: is a type of transport vesicle membrane [GO:0030658]; is a type of Golgi-associated vesicle membrane [GO:0030660]; is_a clathrin-coated vesicle membrane [GO:0030665]; is part of trans-Golgi network transport vesicle [GO:0030140] Also known as: TGN transport vesicle membrane, trans-Golgi network constitutive secretory pathway transport vesicle membrane